{
  "term_label": "Unknown biological process",
  "gene_symbol": "CLDND1",
  "gene": "UniProtKB:Q9NY35",
  "term_id": "UNKNOWN:0002",
  "gene_name": "Claudin domain-containing protein 1"
}